{
  "term_id": "GO:0008543",
  "term_label": "fibroblast growth factor receptor signaling pathway",
  "gene_name": "Fibroblast growth factor 8",
  "gene": "UniProtKB:P55075",
  "gene_symbol": "FGF8"
}